{
  "gene_symbol": "GDPD3",
  "term_id": "GO:0005789",
  "term_label": "endoplasmic reticulum membrane",
  "gene_name": "Lysophospholipase D GDPD3",
  "gene": "UniProtKB:Q7L5L3"
}